(S)-norcoclaurine synthase activity [GO:0050474] (molecular function) Relationships: is a type of hydrolase activity, acting on carbon-nitrogen (but not peptide) bonds [GO:0016810] Also known as: (S)-norlaudanosoline synthase activity, 4-hydroxyphenylacetaldehyde hydro-lyase (adding dopamine), 4-hydroxyphenylacetaldehyde hydro-lyase [adding dopamine; (S)-norcoclaurine-forming] Definition: Catalysis of the reaction: 4-(2-aminoethyl)benzene-1,2-diol + 4-hydroxyphenylacetaldehyde = (S)-norcoclaurine + H2O. Sources: RHEA:16173